isochorismate pyruvate lyase activity [GO:0043904] (molecular function) Relationships: is a type of GO:0016835 Definition: Catalysis of the reaction: isochorismate = salicylate + pyruvate. References: PMID:16248620 Sources: GOC:jl Also known as: IPL, isochorismate-pyruvate lyase activity